{
  "term_label": "DNA-binding transcription factor activity, RNA polymerase II-specific",
  "gene_symbol": "ZNF689",
  "gene": "UniProtKB:Q96CS4",
  "term_id": "GO:0000981",
  "gene_name": "Zinc finger protein 689"
}